{
  "gene_symbol": "HDAC7",
  "term_label": "cytoplasm",
  "term_id": "GO:0005737",
  "gene_name": "Histone deacetylase 7",
  "gene": "UniProtKB:Q8WUI4"
}